{
  "term_label": "intracellular signal transduction",
  "gene": "UniProtKB:Q9Y4K4",
  "gene_symbol": "MAP4K5",
  "gene_name": "Mitogen-activated protein kinase kinase kinase kinase 5",
  "term_id": "GO:0035556"
}